regulation of synaptic signaling by nitric oxide [GO:0150045] (biological process) Definition: Any process that modulates the frequency, rate or extent of synaptic signaling by nitric oxide. References: PMID:26311509 Sources: GOC:aruk, GOC:bc Relationships: is a type of GO:0010646; is_a regulation of signaling [GO:0023051]; regulates GO:0099163